{
  "gene_name": "WAP, Kazal, immunoglobulin, Kunitz and NTR domain-containing protein 1",
  "term_label": "transforming growth factor beta receptor signaling pathway",
  "gene_symbol": "WFIKKN1",
  "gene": "UniProtKB:Q96NZ8",
  "term_id": "GO:0007179"
}